{
  "gene_name": "Olfactory receptor 4X1",
  "term_id": "GO:0005886",
  "term_label": "plasma membrane",
  "gene_symbol": "OR4X1",
  "gene": "UniProtKB:Q8NH49"
}